{
  "gene": "UniProtKB:Q99935",
  "gene_name": "Opiorphin prepropeptide",
  "term_label": "endopeptidase inhibitor activity",
  "term_id": "GO:0004866",
  "gene_symbol": "OPRPN"
}